{
  "gene_name": "Signal recognition particle 19 kDa protein",
  "gene_symbol": "SRP19",
  "gene": "UniProtKB:P09132",
  "term_id": "GO:0008312",
  "term_label": "7S RNA binding"
}